{
  "term_label": "Unknown biological process",
  "gene_symbol": "VCPKMT",
  "gene_name": "Protein N-lysine methyltransferase METTL21D",
  "gene": "UniProtKB:Q9H867",
  "term_id": "UNKNOWN:0002"
}